negative regulation of thrombin-activated receptor signaling pathway [GO:0070495] (biological process) Relationships: is a type of negative regulation of G protein-coupled receptor signaling pathway [GO:0045744]; is a type of regulation of thrombin-activated receptor signaling pathway [GO:0070494]; negatively regulates thrombin-activated receptor signaling pathway [GO:0070493] Sources: GOC:mah Definition: Any process that stops, prevents, or reduces the frequency, rate or extent of thrombin-activated receptor protein signaling pathway activity. A thrombin receptor signaling pathway is the series of molecular signals generated as a consequence of a thrombin-activated receptor binding to one of its physiological ligands. Also known as: negative regulation of thrombin receptor signaling pathway, negative regulation of thrombin receptor signalling pathway